{
  "term_id": "GO:0043491",
  "gene": "UniProtKB:O00750",
  "gene_symbol": "PIK3C2B",
  "gene_name": "Phosphatidylinositol 4-phosphate 3-kinase C2 domain-containing subunit beta",
  "term_label": "phosphatidylinositol 3-kinase/protein kinase B signal transduction"
}